{
  "term_id": "GO:0034650",
  "term_label": "cortisol metabolic process",
  "gene_symbol": "CYP11B2",
  "gene": "UniProtKB:P19099",
  "gene_name": "Cytochrome P450 11B2, mitochondrial"
}